{
  "gene": "UniProtKB:P20273",
  "term_label": "regulation of B cell proliferation",
  "term_id": "GO:0030888",
  "gene_symbol": "CD22",
  "gene_name": "B-cell receptor CD22"
}